vacuolar sequestering of sodium ion [GO:0043182] (biological process) Also known as: sequestering of sodium ion (Na+) in vacuole, sequestration of sodium ion (Na+) in vacuole, sodium ion (Na+) retention in vacuole, sodium ion (Na+) storage in vacuole, vacuolar sequestering of sodium ion (Na+), vacuolar sequestration of sodium ion (Na+), vacuolar sodium ion (Na+) retention, vacuolar sodium ion (Na+) storage Definition: The process of transporting sodium ions into, and confining within, a vacuole. Relationships: is a type of vacuolar sequestering [GO:0043181]; is part of intracellular sodium ion homeostasis [GO:0006883] Sources: GOC:jl